{
  "term_id": "UNKNOWN:0002",
  "gene_symbol": "PRR29",
  "gene": "UniProtKB:P0C7W0",
  "term_label": "Unknown biological process",
  "gene_name": "Proline-rich protein 29"
}